{
  "term_id": "UNKNOWN:0001",
  "gene_symbol": "SPIN2A",
  "term_label": "Unknown molecular function",
  "gene_name": "Spindlin-2A",
  "gene": "UniProtKB:Q99865"
}